{
  "gene_symbol": "RIDA",
  "gene": "UniProtKB:P52758",
  "term_label": "negative regulation of translation",
  "gene_name": "2-iminobutanoate_2-iminopropanoate deaminase",
  "term_id": "GO:0017148"
}